{
  "term_label": "nucleus",
  "gene_name": "RING finger protein 37",
  "gene_symbol": "UBOX5",
  "term_id": "GO:0005634",
  "gene": "UniProtKB:O94941"
}